{
  "gene_name": "Transmembrane protein 19",
  "term_id": "GO:0016020",
  "term_label": "membrane",
  "gene": "UniProtKB:Q96HH6",
  "gene_symbol": "TMEM19"
}